protein localization to non-motile cilium [GO:0097499] (biological process) References: PMID:23128241 Sources: GOC:cilia, GOC:kmv Relationships: is a type of protein localization to cilium [GO:0061512] Also known as: protein localization to nonmotile primary cilium Definition: A process in which a protein is transported to, or maintained in, a location within a non-motile cilium. Subtypes: receptor localization to non-motile cilium [GO:0097500], GO:1903546, GO:1903621